{
  "gene": "UniProtKB:P23109",
  "term_id": "GO:0006188",
  "gene_symbol": "AMPD1",
  "gene_name": "AMP deaminase 1",
  "term_label": "IMP biosynthetic process"
}